{
  "gene_name": "Nuclear pore complex-interacting protein family member B9",
  "gene": "UniProtKB:F8W1W9",
  "term_label": "Unknown cellular component",
  "term_id": "UNKNOWN:0003",
  "gene_symbol": "NPIPB9"
}